acetate biosynthetic process from carbon monoxide [GO:0019415] (biological process) Also known as: acetate anabolism from carbon monoxide, acetate formation from carbon monoxide, acetate synthesis from carbon monoxide, carbon monoxide dehydrogenase pathway Definition: The chemical reactions and pathways resulting in the formation of acetate from other compounds, including carbon monoxide. Sources: GOC:go_curators Relationships: is a type of acetate biosynthetic process [GO:0019413]